{
  "gene_symbol": "SLC17A3",
  "gene": "UniProtKB:O00476",
  "term_id": "GO:0008308",
  "term_label": "voltage-gated monoatomic anion channel activity",
  "gene_name": "Sodium-dependent phosphate transport protein 4"
}